maintenance of protease location in mast cell secretory granule [GO:0033373] (biological process) Relationships: is a type of maintenance of protein location in mast cell secretory granule [GO:0033370]; is part of protease localization to mast cell secretory granule [GO:0033368] Also known as: mast cell protease retention, maintenance of protease localization in mast cell secretory granule Definition: A process in which a protease is maintained in a secretory granule in a mast cell and prevented from moving elsewhere. Sources: GOC:dph, GOC:mah, GOC:tb